integrin alphav-beta5 complex [GO:0034684] (cellular component) Also known as: alphav-beta5 integrin complex, ITGAV-ITGB5 complex Relationships: is_a GO:0008305 References: PMID:12297042 Definition: An integrin complex that comprises one alphav subunit and one beta5 subunit.